{
  "gene": "UniProtKB:P09488",
  "term_id": "UNKNOWN:0003",
  "term_label": "Unknown cellular component",
  "gene_symbol": "GSTM1",
  "gene_name": "Glutathione S-transferase Mu 1"
}